{
  "gene": "UniProtKB:Q8WXX5",
  "term_id": "GO:0031072",
  "gene_name": "DnaJ homolog subfamily C member 9",
  "term_label": "heat shock protein binding",
  "gene_symbol": "DNAJC9"
}